{
  "term_id": "GO:0005847",
  "term_label": "mRNA cleavage and polyadenylation specificity factor complex",
  "gene": "UniProtKB:Q9H0L4",
  "gene_name": "Cleavage stimulation factor subunit 2 tau variant",
  "gene_symbol": "CSTF2T"
}